transcription regulator activator activity [GO:0140537] (molecular function) Note: Usage guidance: transcription regulator activators bind to a transcription regulator to allow it to reach the chromatin or to contact other transcriptional regulators. This activity does not occur at the promoter. For activities that do occur at the promoter, consider GO:0001216 ; DNA-binding transcription activator activity or GO:0003713; transcription coactivator activity; those activities respectively bind DNA themselves or positively regulate a transcription regulator when it is located at the chromatin. References: PMID:9597751 Relationships: is a type of molecular function activator activity [GO:0140677]; is part of regulation of gene expression [GO:0010468]; positively regulates GO:0140110 Definition: A molecular function regulator that increases the activity of a transcription regulator via direct binding and/or post-translational modification.